negative regulation of metabolic process [GO:0009892] (biological process) Definition: Any process that stops, prevents, or reduces the frequency, rate or extent of the chemical reactions and pathways within a cell or an organism. Sources: GOC:go_curators Also known as: down regulation of metabolic process, down-regulation of metabolic process, downregulation of metabolic process, negative regulation of metabolism, negative regulation of organismal metabolism, inhibition of metabolic process, inhibition of organismal metabolic process, negative regulation of multicellular organismal metabolic process Relationships: is a type of regulation of metabolic process [GO:0019222]; is a type of negative regulation of cellular process [GO:0048523]; negatively regulates metabolic process [GO:0008152] Subtypes: negative regulation of biosynthetic process [GO:0009890], negative regulation of catabolic process [GO:0009895], negative regulation of phosphorus metabolic process [GO:0010563], negative regulation of macromolecule metabolic process [GO:0010605], negative regulation of collagen metabolic process [GO:0010713], negative regulation of anthocyanin metabolic process [GO:0031538], negative regulation of hormone metabolic process [GO:0032351], negative regulation of amine metabolic process [GO:0033239], GO:0034249, negative regulation of melanization defense response [GO:0035009], negative regulation of metabolic activity involved in hibernation [GO:0044250], negative regulation of amino acid metabolic process [GO:0045763], negative regulation of lipid metabolic process [GO:0045833], negative regulation of carbohydrate metabolic process [GO:0045912], negative regulation of nucleobase-containing compound metabolic process [GO:0045934], negative regulation of respiratory burst [GO:0060268], GO:0062014, negative regulation of organofluorine metabolic process [GO:0090350], negative regulation of cobalamin metabolic process [GO:0106122], negative regulation of cold-induced thermogenesis [GO:0120163], GO:1901003, negative regulation of cellular respiration [GO:1901856], negative regulation of nitrogen cycle metabolic process [GO:1903315], negative regulation of siRNA processing [GO:1903704], negative regulation of bioluminescence [GO:1905086], GO:1905156, GO:2000378